{
  "term_id": "GO:0008013",
  "gene_name": "Cadherin-19",
  "gene": "UniProtKB:Q9H159",
  "gene_symbol": "CDH19",
  "term_label": "beta-catenin binding"
}